{
  "gene_name": "YEATS domain-containing protein 4",
  "gene": "UniProtKB:O95619",
  "term_id": "GO:0005634",
  "term_label": "nucleus",
  "gene_symbol": "YEATS4"
}